regulation of buoyancy [GO:0031413] (biological process) Sources: GOC:mah, PATO:0001420 Relationships: is a type of biological regulation [GO:0065007] Also known as: buoyancy regulation Definition: Any process that modulates an organism's tendency or ability to rise or float in a fluid medium such as water or air, often through the use of stored gases.